{
  "term_label": "response to hydrogen peroxide",
  "gene_symbol": "CAT",
  "gene": "UniProtKB:P04040",
  "term_id": "GO:0042542",
  "gene_name": "Catalase"
}